lactoferrin transmembrane transporter activity [GO:0033569] (molecular function) Definition: Enables the transfer of lactoferrin from one side of a membrane to the other. Relationships: is a type of protein transmembrane transporter activity [GO:0008320]; is part of GO:0033571 Sources: GOC:mlg